{
  "gene_symbol": "KSR1",
  "gene_name": "Kinase suppressor of Ras 1",
  "term_label": "protein kinase activity",
  "term_id": "GO:0004672",
  "gene": "UniProtKB:Q8IVT5"
}